{
  "term_label": "isoprenoid biosynthetic process",
  "gene_symbol": "PDSS1",
  "gene": "UniProtKB:Q5T2R2",
  "term_id": "GO:0008299",
  "gene_name": "All trans-polyprenyl-diphosphate synthase PDSS1"
}